transcription by RNA polymerase III [GO:0006383] (biological process) References: PMID:12381659 Sources: GOC:jl, GOC:txnOH Regulation: regulated by regulation of transcription by RNA polymerase III [GO:0006359]; negatively regulated by negative regulation of transcription by RNA polymerase III [GO:0016480]; positively regulated by positive regulation of transcription by RNA polymerase III [GO:0045945] Also known as: transcription from Pol III promoter, transcription from RNA polymerase III promoter, U2 snRNA transcription (S. cerevisiae), U6 snRNA transcription (mammalian), transcription from RNA polymerase III type 2 promoter, transcription from RNA polymerase III type 3 promoter, transcription from a RNA polymerase III hybrid type promoter, RNA polymerase III transcription factor activity Subtypes: GO:0001014, GO:0042791, snRNA transcription by RNA polymerase III [GO:0042796], tRNA transcription by RNA polymerase III [GO:0042797] Relationships: is a type of DNA-templated transcription [GO:0006351] Definition: The synthesis of RNA from a DNA template by RNA polymerase III, originating at an RNAP III promoter.